{
  "term_label": "neuropeptide hormone activity",
  "term_id": "GO:0005184",
  "gene_symbol": "SPX",
  "gene": "UniProtKB:Q9BT56",
  "gene_name": "Spexin"
}